{
  "gene_symbol": "LPGAT1",
  "term_id": "GO:0005783",
  "gene": "UniProtKB:Q92604",
  "term_label": "endoplasmic reticulum",
  "gene_name": "Acyl-CoA:lysophosphatidylglycerol acyltransferase 1"
}